{
  "term_label": "Unknown biological process",
  "gene": "UniProtKB:Q96IX9",
  "term_id": "UNKNOWN:0002",
  "gene_name": "Putative ankyrin repeat domain-containing protein 26-like 1",
  "gene_symbol": "ANKRD36BP1"
}